dTDP-dihydrostreptose-streptidine-6-phosphate dihydrostreptosyltransferase activity [GO:0047282] (molecular function) Also known as: dTDP-L-dihydrostreptose:streptidine-6-phosphate dihydrostreptosyltransferase activity, dTDPdihydrostreptose-streptidine-6-phosphate dihydrostreptosyltransferase activity, thymidine diphosphodihydrostreptose-streptidine 6-phosphate dihydrostreptosyltransferase activity Sources: EC:2.4.2.27, RHEA:24392 Relationships: is a type of pentosyltransferase activity [GO:0016763] Definition: Catalysis of the reaction: dTDP-L-dihydrostreptose + streptidine 6-phosphate = O-(1->4)-alpha-L-dihydrostreptosyl-streptidine 6-phosphate + dTDP + H+.